{
  "gene_name": "Neutral and basic amino acid transport protein rBAT",
  "gene": "UniProtKB:Q07837",
  "term_id": "UNKNOWN:0003",
  "term_label": "Unknown cellular component",
  "gene_symbol": "SLC3A1"
}